{
  "gene_symbol": "LARGE1",
  "gene_name": "Xylosyl- and glucuronyltransferase LARGE1",
  "term_label": "glucuronosyltransferase activity",
  "term_id": "GO:0015020",
  "gene": "UniProtKB:O95461"
}